{
  "term_id": "GO:0005737",
  "gene_name": "Caspase recruitment domain-containing protein 9",
  "term_label": "cytoplasm",
  "gene_symbol": "CARD9",
  "gene": "UniProtKB:Q9H257"
}